{
  "term_label": "endocytosis",
  "gene_name": "Unconventional myosin-If",
  "gene_symbol": "MYO1F",
  "term_id": "GO:0006897",
  "gene": "UniProtKB:O00160"
}